{
  "term_label": "Unknown cellular component",
  "term_id": "UNKNOWN:0003",
  "gene": "UniProtKB:Q8TED1",
  "gene_name": "Probable glutathione peroxidase 8",
  "gene_symbol": "GPX8"
}